{
  "term_id": "UNKNOWN:0001",
  "gene_name": "T cell receptor alpha variable 10",
  "gene": "UniProtKB:A0A0B4J240",
  "term_label": "Unknown molecular function",
  "gene_symbol": "TRAV10"
}